alphav-beta3 integrin-vitronectin complex [GO:0071062] (cellular component) Relationships: is a type of plasma membrane protein complex [GO:0098797] References: PMID:10835423 Also known as: ITGAV-ITGB3-VTN complex Definition: A protein complex that consists of an alphav-beta3 integrin complex bound to vitronectin.